membrane invagination [GO:0010324] (biological process) Regulation: regulated by regulation of membrane invagination [GO:1905153]; negatively regulated by negative regulation of membrane invagination [GO:1905154]; positively regulated by positive regulation of membrane invagination [GO:1905155] Definition: The infolding of a membrane. Subtypes: GO:0061736, GO:0099024 Relationships: is a type of GO:0061024 Sources: GOC:tb Also known as: single-organism membrane invagination